selenoneine biosynthetic process [GO:1903257] (biological process) Relationships: is a type of GO:0006578; is a type of modified histidine biosynthetic process [GO:0052703] References: PMID:24828577 Sources: GOC:TermGenie, GO_REF:0000068 Also known as: selenoneine anabolism, selenoneine biosynthesis, selenoneine formation, selenoneine synthesis, L-selenoneine biosynthetic process Definition: The chemical reactions and pathways resulting in the formation of selenoneine.